N-terminal peptidyl-serine dimethylation [GO:0035572] (biological process) Relationships: is a type of N-terminal peptidyl-serine methylation [GO:0035570] Definition: The dimethylation of the N-terminal serine of proteins to form the derivative N,N-dimethylserine. References: PMID:20668449